{
  "gene_name": "X antigen family member 3",
  "gene_symbol": "XAGE3",
  "term_id": "UNKNOWN:0001",
  "gene": "UniProtKB:Q8WTP9",
  "term_label": "Unknown molecular function"
}